{
  "gene_name": "Ly-6_neurotoxin-like protein 1",
  "gene_symbol": "LYNX1",
  "term_id": "GO:0005886",
  "gene": "UniProtKB:P0DP58",
  "term_label": "plasma membrane"
}